{
  "term_id": "GO:0008076",
  "gene": "UniProtKB:Q09470",
  "gene_symbol": "KCNA1",
  "term_label": "voltage-gated potassium channel complex",
  "gene_name": "Potassium voltage-gated channel subfamily A member 1"
}